{
  "gene_name": "G1_S-specific cyclin-E2",
  "term_label": "cyclin E1-CDK2 complex",
  "term_id": "GO:0097134",
  "gene": "UniProtKB:O96020",
  "gene_symbol": "CCNE2"
}